{
  "term_label": "Unknown molecular function",
  "gene_name": "Myotubularin-related protein 11",
  "gene_symbol": "MTMR11",
  "gene": "UniProtKB:A4FU01",
  "term_id": "UNKNOWN:0001"
}